{
  "gene_symbol": "TERF2",
  "gene_name": "Telomeric repeat-binding factor 2",
  "term_label": "telomeric D-loop disassembly",
  "term_id": "GO:0061820",
  "gene": "UniProtKB:Q15554"
}